melatonin biosynthetic process [GO:0030187] (biological process) Sources: GOC:mah, ISBN:0198506732 Definition: The chemical reactions and pathways resulting in the formation of melatonin (N-acetyl-5-methoxytryptamine). Also known as: melatonin anabolism, melatonin biosynthesis, melatonin formation, melatonin synthesis Relationships: is a type of melatonin metabolic process [GO:0030186]; is a type of indole-containing compound biosynthetic process [GO:0042435]; is a type of hormone biosynthetic process [GO:0042446]; is_a amide biosynthetic process [GO:0043604]